{
  "gene_name": "Malonate--CoA ligase ACSF3, mitochondrial",
  "gene_symbol": "ACSF3",
  "term_label": "fatty acid biosynthetic process",
  "term_id": "GO:0006633",
  "gene": "UniProtKB:Q4G176"
}